regulation of fibroblast growth factor receptor signaling pathway involved in neural plate anterior/posterior pattern formation [GO:2000313] (biological process) Subtypes: negative regulation of fibroblast growth factor receptor signaling pathway involved in neural plate anterior/posterior pattern formation [GO:2000314], positive regulation of fibroblast growth factor receptor signaling pathway involved in neural plate anterior/posterior pattern formation [GO:2000315] Sources: GOC:BHF Relationships: is a type of GO:0040036; regulates fibroblast growth factor receptor signaling pathway involved in neural plate anterior/posterior pattern formation [GO:0060825] Definition: Any process that modulates the frequency, rate or extent of fibroblast growth factor receptor signaling pathway involved in neural plate anterior/posterior pattern formation. Also known as: regulation of fibroblast growth factor receptor signalling pathway involved in neural plate anterior/posterior pattern formation